{
  "term_label": "Unknown cellular component",
  "gene_symbol": "ADPRHL1",
  "term_id": "UNKNOWN:0003",
  "gene_name": "Inactive ADP-ribosyltransferase ARH2",
  "gene": "UniProtKB:Q8NDY3"
}